{
  "gene_name": "Kinesin-like protein KIF23",
  "term_label": "kinesin complex",
  "gene_symbol": "KIF23",
  "term_id": "GO:0005871",
  "gene": "UniProtKB:Q02241"
}